{
  "term_label": "Unknown biological process",
  "gene_symbol": "TEX13D",
  "gene": "UniProtKB:A0A0J9YY54",
  "gene_name": "Testis-expressed protein 13D",
  "term_id": "UNKNOWN:0002"
}